protein histidyl modification to diphthamide [GO:0017183] (biological process) Also known as: peptidyl-diphthamide anabolism from peptidyl-histidine, peptidyl-diphthamide biosynthetic process from peptidyl-histidine, peptidyl-diphthamide formation from peptidyl-histidine, peptidyl-diphthamide synthesis from peptidyl-histidine References: PMID:20559380 Sources: GOC:pde Relationships: is a type of peptidyl-histidine modification [GO:0018202] Definition: The modification of peptidyl-histidine to 2'-(3-carboxamido-3-(trimethylammonio)propyl)-L-histidine, known as diphthamide, found in translation elongation factor EF-2. The process occurs in eukaryotes and archaea but not eubacteria.